oxidoreductase activity, acting on a sulfur group of donors [GO:0016667] (molecular function) Relationships: is a type of GO:0016491 Definition: Catalysis of an oxidation-reduction (redox) reaction in which a sulfur-containing group acts as a hydrogen or electron donor and reduces a hydrogen or electron acceptor. Also known as: oxidoreductase activity, acting on sulphur group of donors, oxidoreductase activity, acting on sulfur group of donors, other acceptors Sources: EC:1.8.-.-, GOC:ai Subtypes: dimethyl sulfoxide reductase activity [GO:0009389], adenylyl-sulfate reductase activity [GO:0009973], disulfide oxidoreductase activity [GO:0015036], sulfite reductase activity [GO:0016002], oxidoreductase activity, acting on a sulfur group of donors, NAD(P) as acceptor [GO:0016668], oxidoreductase activity, acting on a sulfur group of donors, cytochrome as acceptor [GO:0016669], GO:0016670, GO:0016671, oxidoreductase activity, acting on a sulfur group of donors, quinone or similar compound as acceptor [GO:0016672], oxidoreductase activity, acting on a sulfur group of donors, iron-sulfur protein as acceptor [GO:0016673], sulfiredoxin activity [GO:0032542], NADPH:sulfur oxidoreductase activity [GO:0043914], CoB--CoM heterodisulfide reductase activity [GO:0051912], reduced coenzyme F420:heterodisulfide oxidoreductase activity [GO:0052752], sulfite reductase (coenzyme F420) activity [GO:0052806], aflatoxin reductase (coenzyme F420) activity [GO:0052807], sulfur:ferric ion oxidoreductase activity [GO:0070226]